{
  "term_label": "Unknown biological process",
  "gene_symbol": "AKR1B1",
  "gene_name": "Aldo-keto reductase family 1 member B1",
  "term_id": "UNKNOWN:0002",
  "gene": "UniProtKB:P15121"
}